{
  "gene_name": "Atlastin-2",
  "gene": "UniProtKB:Q8NHH9",
  "term_id": "GO:0051260",
  "gene_symbol": "ATL2",
  "term_label": "protein homooligomerization"
}